disordered domain specific binding [GO:0097718] (molecular function) Definition: Binding to a disordered domain of a protein. References: PMID:11746698 Sources: GOC:gg Relationships: is a type of GO:0019904 Also known as: disordered protein domain specific binding